{
  "gene": "UniProtKB:P28066",
  "term_id": "GO:0019773",
  "term_label": "proteasome core complex, alpha-subunit complex",
  "gene_symbol": "PSMA5",
  "gene_name": "Proteasome subunit alpha type-5"
}